{
  "term_label": "formation of translation preinitiation complex",
  "term_id": "GO:0001731",
  "gene_name": "Density-regulated protein",
  "gene": "UniProtKB:O43583",
  "gene_symbol": "DENR"
}